{
  "gene": "UniProtKB:P48745",
  "gene_name": "CCN family member 3",
  "gene_symbol": "CCN3",
  "term_label": "signal transduction",
  "term_id": "GO:0007165"
}